{
  "gene": "UniProtKB:O94953",
  "term_label": "nucleus",
  "gene_name": "Lysine-specific demethylase 4B",
  "term_id": "GO:0005634",
  "gene_symbol": "KDM4B"
}